protein linear deubiquitination [GO:1990108] (biological process) References: PMID:23708998 Relationships: is a type of protein deubiquitination [GO:0016579] Definition: A protein deubiquitination process in which a linear polymer of ubiquitin, formed by the amino-terminal methionine (M1) of one ubiquitin molecule and by the carboxy-terminal glycine (G76) of the next, is removed from a protein.